carnitine:O-acyl-L-carnitine antiporter activity [GO:0005476] (molecular function) Relationships: is_a GO:0015226; is a type of O-acyl-L-carnitine transmembrane transporter activity [GO:0015227]; is_a antiporter activity [GO:0015297] References: PMID:9032458 Definition: Catalysis of the reaction: carnitine (mitochondrial) + O-acyl-L-carnitine (cytoplasm) = carnitine (cytoplasm) + O-acyl-L-carnitine (mitochondrial). Also known as: carnitine/acyl carnitine carrier activity, carnitine:acyl carnitine carrier activity, fatty acyl carnitine carrier